{
  "gene_symbol": "CLDN20",
  "gene_name": "Claudin-20",
  "term_label": "Unknown molecular function",
  "gene": "UniProtKB:P56880",
  "term_id": "UNKNOWN:0001"
}